{
  "term_id": "GO:0051604",
  "gene_name": "Serine protease 58",
  "gene_symbol": "PRSS58",
  "term_label": "protein maturation",
  "gene": "UniProtKB:Q8IYP2"
}